{
  "gene_name": "Bax inhibitor 1",
  "gene_symbol": "TMBIM6",
  "gene": "UniProtKB:P55061",
  "term_id": "GO:0005789",
  "term_label": "endoplasmic reticulum membrane"
}